{
  "gene": "UniProtKB:Q8N4V2",
  "gene_name": "Synaptic vesicle 2-related protein",
  "gene_symbol": "SVOP",
  "term_id": "UNKNOWN:0003",
  "term_label": "Unknown cellular component"
}